ABC-type maltose transporter activity [GO:0015423] (molecular function) Definition: Enables the transfer of a solute or solutes from one side of a membrane to the other according to the reaction: ATP + H2O + maltose(out) = ADP + phosphate + maltose(in). Sources: RHEA:22132 Also known as: ABC-type maltose transporter, maltose ABC transporter, ATP-dependent maltose transmembrane transporter activity, ATPase-coupled maltose transmembrane transporter activity, maltooligosaccharide-importing ATPase activity, maltose-transporting ATPase activity Relationships: is a type of maltose transmembrane transporter activity [GO:0005363]; is a type of ABC-type oligosaccharide transporter activity [GO:0015422]; is part of maltose transmembrane transport [GO:1904981]